{
  "gene": "UniProtKB:Q19T08",
  "term_id": "GO:0005829",
  "gene_name": "Endothelial cell-specific chemotaxis regulator",
  "gene_symbol": "ECSCR",
  "term_label": "cytosol"
}